very long-chain fatty acid beta-oxidation [GO:0140493] (biological process) Note: While there is not universal consensus on the lengths of short-, medium-, long- and very-long-chain fatty acids, the GO uses the definitions in ChEBI (see CHEBI:26666, CHEBI:59554, CHEBI:15904 and CHEBI:27283). Definition: A fatty acid beta-oxidation pathway acting on a very long-chain fatty acid. A very long-chain fatty acid has an aliphatic tail containing more than 22 carbons. The partway stars with the conversion of an acyl-CoA to a trans-2-enoyl-CoA, catalyzed by acyl-CoA oxidase; the electrons removed by oxidation pass directly to oxygen and produce hydrogen peroxide, which is cleaved by peroxisomal catalases. Fatty acid beta-oxidation begins with the addition of coenzyme A to a fatty acid, and ends when only two or three carbons remain (as acetyl-CoA or propionyl-CoA respectively). References: PMID:17028011, PMID:32169171 Sources: GOC:ha Relationships: is a type of fatty acid beta-oxidation using acyl-CoA oxidase [GO:0033540]; is a type of very long-chain fatty acid catabolic process [GO:0042760]